{
  "gene": "UniProtKB:O15031",
  "term_id": "GO:0007416",
  "gene_name": "Plexin-B2",
  "gene_symbol": "PLXNB2",
  "term_label": "synapse assembly"
}